{
  "gene_name": "Zinc finger protein 2",
  "gene_symbol": "ZNF2",
  "gene": "UniProtKB:Q9BSG1",
  "term_id": "UNKNOWN:0003",
  "term_label": "Unknown cellular component"
}